{
  "term_id": "GO:0005886",
  "gene_symbol": "CNRIP1",
  "gene": "UniProtKB:Q96F85",
  "gene_name": "CB1 cannabinoid receptor-interacting protein 1",
  "term_label": "plasma membrane"
}